{
  "term_label": "2',3'-cyclic-nucleotide 3'-phosphodiesterase activity",
  "term_id": "GO:0004113",
  "gene_name": "2',3'-cyclic-nucleotide 3'-phosphodiesterase",
  "gene": "UniProtKB:P09543",
  "gene_symbol": "CNP"
}